{
  "term_label": "Unknown cellular component",
  "term_id": "UNKNOWN:0003",
  "gene": "UniProtKB:Q13572",
  "gene_name": "Inositol-tetrakisphosphate 1-kinase",
  "gene_symbol": "ITPK1"
}